{
  "gene_symbol": "CNTNAP3",
  "term_label": "Unknown molecular function",
  "gene_name": "Contactin-associated protein-like 3",
  "gene": "UniProtKB:Q9BZ76",
  "term_id": "UNKNOWN:0001"
}